{
  "term_label": "interstrand cross-link repair",
  "term_id": "GO:0036297",
  "gene_name": "DNA cross-link repair 1A protein",
  "gene": "UniProtKB:Q6PJP8",
  "gene_symbol": "DCLRE1A"
}